{
  "term_label": "lipid transport",
  "gene_symbol": "ABCA4",
  "gene_name": "Retinal-specific phospholipid-transporting ATPase ABCA4",
  "gene": "UniProtKB:P78363",
  "term_id": "GO:0006869"
}